{
  "gene_name": "tRNA-splicing endonuclease subunit Sen2",
  "gene": "UniProtKB:Q8NCE0",
  "gene_symbol": "TSEN2",
  "term_id": "GO:0000379",
  "term_label": "tRNA-type intron splice site recognition and cleavage"
}